chitosome membrane [GO:0030661] (cellular component) Relationships: is a type of cytoplasmic vesicle membrane [GO:0030659]; is a type of bounding membrane of organelle [GO:0098588]; is part of chitosome [GO:0045009] Definition: The lipid bilayer surrounding a chitosome. Sources: GOC:mah